{
  "gene_symbol": "PTPRR",
  "term_id": "GO:0005829",
  "term_label": "cytosol",
  "gene": "UniProtKB:Q15256",
  "gene_name": "Receptor-type tyrosine-protein phosphatase R"
}